{
  "gene": "UniProtKB:Q9UID6",
  "gene_name": "Zinc finger protein 639",
  "gene_symbol": "ZNF639",
  "term_id": "GO:0000978",
  "term_label": "RNA polymerase II cis-regulatory region sequence-specific DNA binding"
}